negative regulation of nematode pharyngeal pumping [GO:1903745] (biological process) Relationships: is a type of regulation of nematode pharyngeal pumping [GO:0043051]; is a type of GO:1903999; negatively regulates nematode pharyngeal pumping [GO:0043050] Definition: Any process that stops, prevents or reduces the frequency, rate or extent of nematode pharyngeal pumping. Also known as: down regulation of pharyngeal pumping, down-regulation of pharyngeal pumping, downregulation of pharyngeal pumping, inhibition of pharyngeal pumping, down regulation of pumping behavior, down-regulation of pumping behavior, downregulation of pumping behavior, inhibition of pumping behavior, negative regulation of pumping behavior References: PMID:25329901 Sources: GOC:TermGenie, GOC:kmv, GO_REF:0000058